{
  "term_label": "plasma membrane",
  "gene_name": "Vesicle-associated membrane protein-associated protein B_C",
  "gene_symbol": "VAPB",
  "gene": "UniProtKB:O95292",
  "term_id": "GO:0005886"
}